{
  "gene": "UniProtKB:Q8NA23",
  "term_label": "Unknown cellular component",
  "term_id": "UNKNOWN:0003",
  "gene_symbol": "WDR31",
  "gene_name": "WD repeat-containing protein 31"
}